{
  "gene": "UniProtKB:Q9BRL6",
  "term_id": "GO:0016607",
  "gene_symbol": "SRSF8",
  "gene_name": "Serine_arginine-rich splicing factor 8",
  "term_label": "nuclear speck"
}